exit from mitosis [GO:0010458] (biological process) Sources: GOC:dph, GOC:tb Also known as: exit from mitotic division, mitotic exit Regulation: negatively regulated by GO:0001100; regulated by regulation of exit from mitosis [GO:0007096]; positively regulated by GO:0031536 Definition: The cell cycle transition where a cell leaves M phase and enters a new G1 phase. M phase is the part of the mitotic cell cycle during which mitosis and cytokinesis take place. Relationships: is a type of mitotic cell cycle phase transition [GO:0044772]; is part of mitotic nuclear division [GO:0140014]